{
  "gene_name": "Integrin beta-8",
  "gene_symbol": "ITGB8",
  "gene": "UniProtKB:P26012",
  "term_id": "GO:0005925",
  "term_label": "focal adhesion"
}